{
  "term_id": "GO:0008236",
  "gene_symbol": "TMPRSS11B",
  "term_label": "serine-type peptidase activity",
  "gene": "UniProtKB:Q86T26",
  "gene_name": "Transmembrane protease serine 11B"
}